{
  "gene_symbol": "ST7L",
  "gene_name": "Suppressor of tumorigenicity 7 protein-like",
  "gene": "UniProtKB:Q8TDW4",
  "term_id": "UNKNOWN:0002",
  "term_label": "Unknown biological process"
}